DRM complex [GO:0070176] (CC) Relationships: is a type of RNA polymerase II transcription repressor complex [GO:0090571] References: PMID:17075059 Also known as: DP/Rb/MuvB Definition: A transcriptional repressor complex that contains the lin-9, lin-35, lin-37, lin-52, lin-53, lin-5is involved in 4-, dpl-1 and efl-1 proteins, and is involved in cell fate specification.